{
  "gene": "UniProtKB:O14602",
  "term_label": "cytoplasm",
  "gene_name": "Eukaryotic translation initiation factor 1A, Y-chromosomal",
  "gene_symbol": "EIF1AY",
  "term_id": "GO:0005737"
}